{
  "term_label": "adenylate cyclase-activating G protein-coupled receptor signaling pathway",
  "term_id": "GO:0007189",
  "gene_name": "Urocortin-2",
  "gene_symbol": "UCN2",
  "gene": "UniProtKB:Q96RP3"
}